response to differentiation-inducing factor 2 [GO:1905960] (biological process) Subtypes: GO:0061862 Relationships: is_a response to ether [GO:0045472]; is a type of response to ketone [GO:1901654] Definition: Any process that results in a change in state or activity of a cell or an organism (in terms of movement, secretion, enzyme production, gene expression, etc.) as a result of a 1-(3,5-dichloro-2,6-dihydroxy-4-methoxyphenyl)pentan-1-one stimulus. Also known as: response to 1-(3,5-dichloro-2,6-dihydroxy-4-methoxyphenyl)pentan-1-one, response to DIF-2, response to DIF2 References: PMID:19684855, PMID:3355503 Sources: GOC:TermGenie, GOC:rjd, GO_REF:0000071